positive regulation of protein localization [GO:1903829] (biological process) Subtypes: positive regulation of protein transport [GO:0051222], GO:0110083, positive regulation of protein localization to chromatin [GO:0120187], positive regulation of protein localization to lysosome [GO:0150032], positive regulation of protein localization to cell-cell junction [GO:0150107], positive regulation of protein localization to nucleus [GO:1900182], positive regulation of protein localization to spindle pole body [GO:1902365], positive regulation of protein localization to synapse [GO:1902474], positive regulation of protein localization to cell tip [GO:1903068], positive regulation of protein localization to cilium [GO:1903566], positive regulation of protein localization to cell periphery [GO:1904377], positive regulation of protein localization to centrosome [GO:1904781], positive regulation of asymmetric protein localization involved in cell fate determination [GO:1904787], positive regulation of protein localization to chromosome, telomeric region [GO:1904816], positive regulation of protein localization to phagocytic vesicle [GO:1905171], positive regulation of protein localization to kinetochore [GO:1905342], positive regulation of protein localization to membrane [GO:1905477], positive regulation of protein localization to endoplasmic reticulum [GO:1905552], positive regulation of protein localization to endosome [GO:1905668], positive regulation of protein localization to cell leading edge [GO:1905873], GO:2000010 Relationships: is a type of regulation of protein localization [GO:0032880]; is_a positive regulation of biological process [GO:0048518]; positively regulates GO:0008104 Also known as: positive regulation of cellular protein localisation, positive regulation of cellular protein localization, up regulation of cellular protein localisation, up regulation of cellular protein localization, up-regulation of cellular protein localisation, up-regulation of cellular protein localization, upregulation of cellular protein localisation, upregulation of cellular protein localization Definition: Any process that activates or increases the frequency, rate or extent of a protein localization. Sources: GOC:TermGenie, GOC:vw, GO_REF:0000058